{
  "gene_name": "Acylphosphatase-2",
  "term_label": "Unknown biological process",
  "term_id": "UNKNOWN:0002",
  "gene_symbol": "ACYP2",
  "gene": "UniProtKB:P14621"
}